{
  "term_label": "oligosaccharyltransferase complex",
  "gene_name": "Magnesium transporter protein 1",
  "gene": "UniProtKB:Q9H0U3",
  "gene_symbol": "MAGT1",
  "term_id": "GO:0008250"
}